{
  "gene": "UniProtKB:Q9P0U1",
  "gene_symbol": "TOMM7",
  "term_label": "mitochondrial outer membrane translocase complex",
  "term_id": "GO:0005742",
  "gene_name": "Mitochondrial import receptor subunit TOM7 homolog"
}